{
  "term_id": "UNKNOWN:0001",
  "gene": "UniProtKB:O95229",
  "gene_name": "ZW10 interactor",
  "gene_symbol": "ZWINT",
  "term_label": "Unknown molecular function"
}